{
  "term_id": "GO:0005634",
  "gene": "UniProtKB:Q6PJG6",
  "term_label": "nucleus",
  "gene_name": "BRCA1-associated ATM activator 1",
  "gene_symbol": "BRAT1"
}